lateral line nerve glial cell differentiation [GO:0048895] (biological process) References: PMID:12062041 Subtypes: anterior lateral line nerve glial cell differentiation [GO:0048913], posterior lateral line nerve glial cell differentiation [GO:0048931] Definition: The process in which a relatively unspecialized cell acquires specialized features of a glial cell in a lateral line nerve. Relationships: is a type of glial cell differentiation [GO:0010001]; is part of lateral line nerve development [GO:0048892]